{
  "gene_symbol": "SCLY",
  "gene": "UniProtKB:Q96I15",
  "gene_name": "Selenocysteine lyase",
  "term_id": "UNKNOWN:0002",
  "term_label": "Unknown biological process"
}